{
  "term_label": "endocytic vesicle",
  "gene_symbol": "RABGEF1",
  "term_id": "GO:0030139",
  "gene": "UniProtKB:Q9UJ41",
  "gene_name": "Rab5 GDP_GTP exchange factor"
}